{
  "gene_name": "Putative heat shock protein HSP 90-beta-3",
  "gene": "UniProtKB:Q58FF7",
  "gene_symbol": "HSP90AB3P",
  "term_label": "protein folding",
  "term_id": "GO:0006457"
}